{
  "gene_symbol": "NUP62CL",
  "term_id": "UNKNOWN:0002",
  "gene_name": "Nucleoporin-62 C-terminal-like protein",
  "term_label": "Unknown biological process",
  "gene": "UniProtKB:Q9H1M0"
}